{
  "term_label": "immunoglobulin complex",
  "term_id": "GO:0019814",
  "gene": "UniProtKB:A0A0C4DH73",
  "gene_name": "Immunoglobulin kappa variable 1-12",
  "gene_symbol": "IGKV1-12"
}